gonadotropin-releasing hormone binding [GO:0051448] (molecular function) Also known as: GnRH binding, gonadotrophin releasing hormone binding References: PMID:1984190 Sources: GOC:pr Relationships: is a type of GO:0017046 Definition: Binding to gonadotropin-releasing hormone (GnRH), a peptide hormone responsible for the release of follicle-stimulating hormone (FSH) and luteinizing hormone (LH) from the anterior pituitary. GnRH is synthesized and released by the hypothalamus.